{
  "gene_symbol": "OR51L1",
  "gene": "UniProtKB:Q8NGJ5",
  "gene_name": "Olfactory receptor 51L1",
  "term_label": "plasma membrane",
  "term_id": "GO:0005886"
}